{
  "term_label": "bile acid metabolic process",
  "term_id": "GO:0008206",
  "gene_symbol": "SLC27A5",
  "gene_name": "Long-chain fatty acid transport protein 5",
  "gene": "UniProtKB:Q9Y2P5"
}